{
  "term_label": "nucleus",
  "gene_symbol": "CNPPD1",
  "gene_name": "Protein CNPPD1",
  "term_id": "GO:0005634",
  "gene": "UniProtKB:Q9BV87"
}